5-oxopent-3-ene-1,2,5-tricarboxylate decarboxylase activity [GO:0018800] (molecular function) Sources: EC:4.1.1.68 Definition: Catalysis of the reaction: 5-oxopent-3-ene-1,2,5-tricarboxylate = 2-oxohept-3-enedioate + CO2. Also known as: 5-carboxymethyl-2-oxo-hex-3-ene-1,7-dioate decarboxylase activity, OPET decarboxylase activity, 5-carboxymethyl-2-oxo-hex-3-ene-1,6-dioate decarboxylase activity, 5-oxopent-3-ene-1,2,5-tricarboxylate carboxy-lyase (2-oxohept-3-enedioate-forming), 5-oxopent-3-ene-1,2,5-tricarboxylate carboxy-lyase activity, HpaG-2, HpaG2 Relationships: is a type of carboxy-lyase activity [GO:0016831]